uracil dehydrogenase activity [GO:0050383] (molecular function) Relationships: is a type of oxidoreductase activity, acting on CH or CH2 groups [GO:0016725] Definition: Catalysis of the reaction: uracil + acceptor = barbiturate + reduced acceptor. Sources: RHEA:22752